acyl carrier activity [GO:0000036] (molecular function) Also known as: ACP phosphopantetheine attachment site binding involved in fatty acid biosynthetic process Definition: Binding an acyl group and presenting it for processing or offloading to a cognate enzyme. Covalently binds the acyl group via a phosphopantetheine prosthetic group and mediates protein-protein interactions with the enzyme conferring specificity. The acyl carrier protein (ACP) presents substrates to enzymes involved in fatty acid biosynthesis or in polyketide secondary metabolite biosynthesis. Sources: GOC:jl, GOC:vw Relationships: is a type of GO:0044620; is a type of GO:0140414; is part of fatty acid biosynthetic process [GO:0006633]